{
  "gene_name": "DNA polymerase alpha catalytic subunit",
  "gene": "UniProtKB:P09884",
  "term_label": "leading strand elongation",
  "gene_symbol": "POLA1",
  "term_id": "GO:0006272"
}